{
  "term_id": "GO:0005829",
  "gene_name": "All-trans-retinol dehydrogenase [NAD(+)] ADH7",
  "gene_symbol": "ADH7",
  "gene": "UniProtKB:P40394",
  "term_label": "cytosol"
}